{
  "term_id": "GO:0006366",
  "term_label": "transcription by RNA polymerase II",
  "gene": "UniProtKB:P19387",
  "gene_symbol": "POLR2C",
  "gene_name": "DNA-directed RNA polymerase II subunit RPB3"
}